NAD+-dinitrogen-reductase ADP-D-ribosyltransferase activity [GO:0030701] (molecular function) Also known as: ADP-ribosyltransferase activity, NAD-dinitrogen-reductase ADP-D-ribosyltransferase activity, NAD+:[dinitrogen reductase] (ADP-D-ribosyl)transferase activity, NAD--azoferredoxin (ADP-ribose)transferase activity, NAD-azoferredoxin (ADPribose)transferase activity Relationships: is a type of pentosyltransferase activity [GO:0016763] Definition: Catalysis of the reaction: NAD+ + [dinitrogen reductase] = nicotinamide + ADP-D-ribosyl-[dinitrogen reductase]. Sources: EC:2.4.2.37